{
  "gene_symbol": "IL23R",
  "gene": "UniProtKB:Q5VWK5",
  "gene_name": "Interleukin-23 receptor",
  "term_label": "peptide hormone binding",
  "term_id": "GO:0017046"
}